{
  "gene": "UniProtKB:Q9UPU5",
  "gene_name": "Ubiquitin carboxyl-terminal hydrolase 24",
  "term_label": "nucleus",
  "gene_symbol": "USP24",
  "term_id": "GO:0005634"
}